{
  "term_label": "endocytic vesicle",
  "term_id": "GO:0030139",
  "gene": "UniProtKB:Q9UM54",
  "gene_symbol": "MYO6",
  "gene_name": "Unconventional myosin-VI"
}